{
  "term_id": "GO:0006355",
  "gene": "UniProtKB:Q86X55",
  "term_label": "regulation of DNA-templated transcription",
  "gene_name": "Histone-arginine methyltransferase CARM1",
  "gene_symbol": "CARM1"
}